network-forming collagen trimer [GO:0098642] (cellular component) Definition: A collagen trimer that forms networks. References: PMID:21421911 Subtypes: collagen type IV trimer [GO:0005587], collagen type VIII trimer [GO:0005591], collagen type X trimer [GO:0005599] Relationships: is a type of collagen trimer [GO:0005581]; is part of GO:0098645